{
  "gene": "UniProtKB:Q96EC8",
  "term_id": "GO:0005802",
  "gene_symbol": "YIPF6",
  "term_label": "trans-Golgi network",
  "gene_name": "Protein YIPF6"
}